{
  "term_id": "GO:0004674",
  "gene_name": "Testis-specific serine_threonine-protein kinase 1",
  "term_label": "protein serine/threonine kinase activity",
  "gene_symbol": "TSSK1B",
  "gene": "UniProtKB:Q9BXA7"
}